{
  "gene_symbol": "NCK1",
  "term_label": "receptor tyrosine kinase binding",
  "gene_name": "Cytoplasmic protein NCK1",
  "gene": "UniProtKB:P16333",
  "term_id": "GO:0030971"
}